{
  "gene_symbol": "STT3A",
  "term_label": "dolichyl-diphosphooligosaccharide-protein glycotransferase activity",
  "term_id": "GO:0004579",
  "gene_name": "Dolichyl-diphosphooligosaccharide--protein glycosyltransferase subunit STT3A",
  "gene": "UniProtKB:P46977"
}